gamma-tubulin complex localization [GO:0033566] (BP) Definition: Any process in which a gamma-tubulin complex is transported to, or maintained in, a specific location. Sources: GOC:mah Also known as: establishment and maintenance of gamma-tubulin complex localization, gamma-tubulin complex localisation Relationships: is a type of GO:0031503 Subtypes: GO:1990735